regulation of crystal cell differentiation [GO:0042689] (biological process) Definition: Any process that modulates the frequency, rate or extent of crystal cell differentiation. Relationships: is_a GO:0045610; regulates crystal cell differentiation [GO:0042688] Subtypes: negative regulation of crystal cell differentiation [GO:0042690], GO:0042691 Sources: GOC:go_curators